{
  "term_id": "UNKNOWN:0002",
  "gene_symbol": "JMJD8",
  "term_label": "Unknown biological process",
  "gene_name": "JmjC domain-containing protein 8",
  "gene": "UniProtKB:Q96S16"
}